{
  "term_id": "UNKNOWN:0002",
  "gene_name": "C3 and PZP-like alpha-2-macroglobulin domain-containing protein 8",
  "gene": "UniProtKB:Q8IZJ3",
  "gene_symbol": "CPAMD8",
  "term_label": "Unknown biological process"
}